{
  "term_id": "UNKNOWN:0001",
  "gene_symbol": "DAD1",
  "gene": "UniProtKB:P61803",
  "term_label": "Unknown molecular function",
  "gene_name": "Dolichyl-diphosphooligosaccharide--protein glycosyltransferase subunit DAD1"
}